plus-end directed microtubule sliding [GO:0031535] (biological process) Regulation: negatively regulated by negative regulation of plus-end directed microtubule sliding [GO:0062168]; RO_0002211 by regulation of plus-end directed microtubule sliding [GO:0062169] Relationships: is a type of GO:0051012 Sources: GOC:mah, GOC:vw Definition: The movement of one microtubule along another microtubule, where the motion is directed towards the plus ends of the microtubules.